{
  "term_id": "GO:0072686",
  "term_label": "mitotic spindle",
  "gene": "UniProtKB:O95834",
  "gene_name": "Echinoderm microtubule-associated protein-like 2",
  "gene_symbol": "EML2"
}